aeciospore formation [GO:0075247] (biological process) Relationships: is a type of asexual sporulation resulting in formation of a cellular spore [GO:0043936] Regulation: regulated by regulation of aeciospore formation [GO:0075248]; positively regulated by positive regulation of aeciospore formation [GO:0075249]; negatively regulated by negative regulation of aeciospore formation [GO:0075250] Definition: The process in which a dikaryotic spore of typically a rust fungus is produced in an aecium; in heteroecious rusts, the aeciospore is a spore stage that infects the alternate host. Sources: GOC:pamgo_curators